{
  "gene": "UniProtKB:P16619",
  "term_label": "positive regulation of cell migration",
  "term_id": "GO:0030335",
  "gene_name": "C-C motif chemokine 3-like 1",
  "gene_symbol": "CCL3L1"
}